{
  "gene_name": "Uncharacterized protein C14orf132",
  "term_label": "Unknown biological process",
  "term_id": "UNKNOWN:0002",
  "gene": "UniProtKB:Q9NPU4",
  "gene_symbol": "C14orf132"
}